{
  "term_id": "GO:0008191",
  "term_label": "metalloendopeptidase inhibitor activity",
  "gene": "UniProtKB:P01033",
  "gene_name": "Metalloproteinase inhibitor 1",
  "gene_symbol": "TIMP1"
}